{
  "gene": "UniProtKB:O00482",
  "gene_name": "Nuclear receptor subfamily 5 group A member 2",
  "term_label": "RNA polymerase II cis-regulatory region sequence-specific DNA binding",
  "gene_symbol": "NR5A2",
  "term_id": "GO:0000978"
}